{
  "term_label": "Unknown molecular function",
  "term_id": "UNKNOWN:0001",
  "gene_name": "Rab GTPase-binding effector protein 2",
  "gene_symbol": "RABEP2",
  "gene": "UniProtKB:Q9H5N1"
}